chaperone-mediated autophagy translocation complex [GO:0061742] (cellular component) Also known as: CMA translocation complex, CMA receptor complex, chaperone-mediated autophagy receptor complex Relationships: is a type of GO:0098796; is part of GO:0005765 Definition: A lysosomal membrane protein complex that enables the translocation of a target protein across the lysosomal membrane as part of chaperone-mediated autophagy. References: PMID:20797626 Sources: GOC:PARL, GOC:dph, GOC:pad